ubiquitin-dependent protein catabolic process [GO:0006511] (BP) Subtypes: proteasome-mediated ubiquitin-dependent protein catabolic process [GO:0043161], ubiquitin-dependent protein catabolic process via the multivesicular body sorting pathway [GO:0043162] Relationships: is a type of GO:0019941; has part protein ubiquitination [GO:0016567] Definition: The chemical reactions and pathways resulting in the breakdown of a protein or peptide by hydrolysis of its peptide bonds, initiated by the covalent attachment of a ubiquitin group, or multiple ubiquitin groups, to the protein. Sources: GOC:go_curators Regulation: regulated by regulation of ubiquitin-dependent protein catabolic process [GO:2000058]; negatively regulated by negative regulation of ubiquitin-dependent protein catabolic process [GO:2000059]; positively regulated by positive regulation of ubiquitin-dependent protein catabolic process [GO:2000060] Also known as: protein degradation tagging activity, ubiquitin-dependent protein breakdown, ubiquitin-dependent protein catabolism, ubiquitin-dependent protein degradation, ubiquitin-dependent proteolysis, myofibrillar protein ubiquitination during ubiquitin-dependent protein breakdown, myofibrillar protein ubiquitination during ubiquitin-dependent protein catabolic process, myofibrillar protein ubiquitination during ubiquitin-dependent protein catabolism, myofibrillar protein ubiquitination during ubiquitin-dependent protein degradation, protein ubiquitination during ubiquitin-dependent protein breakdown, protein ubiquitination during ubiquitin-dependent protein catabolism, protein ubiquitination during ubiquitin-dependent protein degradation, protein ubiquitinylation during ubiquitin-dependent protein catabolic process, protein ubiquitinylation during ubiquitin-dependent protein catabolism, protein ubiquitylation during ubiquitin-dependent protein catabolic process, protein ubiquitylation during ubiquitin-dependent protein catabolism, protein ubiquitination during ubiquitin-dependent protein catabolic process, protein ubiquitination involved in ubiquitin-dependent protein catabolic process